guanidinoacetate kinase activity [GO:0047973] (molecular function) Definition: Catalysis of the reaction: ATP + guanidinoacetate = ADP + 2 H+ + phosphoguanidinoacetate. Sources: EC:2.7.3.1, RHEA:14145 Also known as: guanidoacetate kinase activity, ATP:guanidinoacetate N-phosphotransferase activity, glycocyamine kinase activity Relationships: is a type of kinase activity [GO:0016301]; is_a phosphotransferase activity, nitrogenous group as acceptor [GO:0016775]